{
  "gene": "UniProtKB:Q13634",
  "gene_symbol": "CDH18",
  "term_id": "GO:0044331",
  "gene_name": "Cadherin-18",
  "term_label": "cell-cell adhesion mediated by cadherin"
}